{
  "gene_name": "Interleukin-1 receptor-associated kinase-like 2",
  "term_label": "nucleus",
  "gene": "UniProtKB:O43187",
  "term_id": "GO:0005634",
  "gene_symbol": "IRAK2"
}